cell wall beta-glucan metabolic process [GO:0034406] (biological process) Definition: The chemical reactions and pathways involving beta-glucans, compounds composed of glucose residues linked by beta-D-glucosidic bonds, found in the walls of cells. Sources: GOC:mah Relationships: is a type of GO:0010383; is a type of beta-glucan metabolic process [GO:0051273] Subtypes: cell wall (1->3)-beta-D-glucan metabolic process [GO:0034407], GO:0034410, plant-type cell wall cellulose metabolic process [GO:0052541], GO:0070879 Also known as: cell wall beta-glucan metabolism